{
  "gene": "UniProtKB:P60763",
  "gene_name": "Ras-related C3 botulinum toxin substrate 3",
  "term_label": "regulation of actin cytoskeleton organization",
  "gene_symbol": "RAC3",
  "term_id": "GO:0032956"
}